old mitotic spindle pole body [GO:0071957] (cellular component) References: PMID:15132994 Sources: GOC:mah, GOC:vw Relationships: is_a GO:0044732 Definition: The spindle pole body that exists in a cell prior to spindle pole body duplication. An old spindle pole body segregates to the daughter cell upon mitosis, and lacks active proteins involved in signaling exit from mitosis. Also known as: old SPB